{
  "term_id": "GO:0038023",
  "term_label": "signaling receptor activity",
  "gene": "UniProtKB:Q6UY18",
  "gene_symbol": "LINGO4",
  "gene_name": "Leucine-rich repeat and immunoglobulin-like domain-containing nogo receptor-interacting protein 4"
}